{
  "term_id": "GO:0006357",
  "term_label": "regulation of transcription by RNA polymerase II",
  "gene_symbol": "REPIN1",
  "gene_name": "Replication initiator 1",
  "gene": "UniProtKB:Q9BWE0"
}